{
  "gene_name": "Uncharacterized protein C3orf62",
  "gene": "UniProtKB:Q6ZUJ4",
  "gene_symbol": "C3orf62",
  "term_id": "UNKNOWN:0001",
  "term_label": "Unknown molecular function"
}